fibroblast growth factor production [GO:0090269] (biological process) Relationships: is a type of cytokine production [GO:0001816] Definition: The appearance of a fibroblast growth factor due to biosynthesis or secretion following a cellular stimulus, resulting in an increase in its intracellular or extracellular levels. Regulation: regulated by GO:0090270; positively regulated by GO:0090271; negatively regulated by negative regulation of fibroblast growth factor production [GO:0090272] Sources: GOC:BHF